{
  "term_label": "FAR/SIN/STRIPAK complex",
  "gene": "UniProtKB:Q9ULQ0",
  "term_id": "GO:0090443",
  "gene_name": "Striatin-interacting protein 2",
  "gene_symbol": "STRIP2"
}